{
  "gene_name": "Trafficking protein particle complex subunit 13",
  "term_label": "Unknown molecular function",
  "gene": "UniProtKB:A5PLN9",
  "gene_symbol": "TRAPPC13",
  "term_id": "UNKNOWN:0001"
}